regulation of smooth muscle cell-matrix adhesion [GO:2000097] (biological process) Relationships: is a type of regulation of cell-matrix adhesion [GO:0001952]; regulates smooth muscle cell-matrix adhesion [GO:0061302] Definition: Any process that modulates the frequency, rate or extent of smooth muscle cell-matrix adhesion. Subtypes: positive regulation of smooth muscle cell-matrix adhesion [GO:1905609], negative regulation of smooth muscle cell-matrix adhesion [GO:2000098] Sources: GOC:BHF